{
  "gene": "UniProtKB:P0C626",
  "term_id": "GO:0005549",
  "gene_symbol": "OR5G3",
  "gene_name": "Olfactory receptor 5G3",
  "term_label": "odorant binding"
}